{
  "gene": "UniProtKB:Q99640",
  "term_label": "protein kinase activity",
  "term_id": "GO:0004672",
  "gene_name": "Membrane-associated tyrosine- and threonine-specific cdc2-inhibitory kinase",
  "gene_symbol": "PKMYT1"
}